{
  "gene_symbol": "EN2",
  "term_id": "GO:0030182",
  "term_label": "neuron differentiation",
  "gene_name": "Homeobox protein engrailed-2",
  "gene": "UniProtKB:P19622"
}